non-sensory hair organization [GO:0035316] (biological process) Definition: A process that is carried out at the cellular level which results in the assembly, arrangement of constituent parts, or disassembly of non-sensory hairs. These hairs are polarized cellular extensions that cover much of the insect epidermis. Also known as: trichome organisation, trichome organization and biogenesis, non-sensory hair organization and biogenesis Note: See also the fly_anatomy.ontology term 'trichome ; FBbt:00004979'. References: PMID:11064425 Sources: GOC:mtg_sensu Subtypes: imaginal disc-derived wing hair organization [GO:0035317] Relationships: is a type of plasma membrane bounded cell projection organization [GO:0120036]; is part of hair cell differentiation [GO:0035315]